{
  "gene_symbol": "PAFAH1B1",
  "term_id": "GO:0043005",
  "gene_name": "Platelet-activating factor acetylhydrolase IB subunit beta",
  "term_label": "neuron projection",
  "gene": "UniProtKB:P43034"
}